{
  "gene_symbol": "TRIM43B",
  "term_id": "GO:0005737",
  "term_label": "cytoplasm",
  "gene": "UniProtKB:A6NCK2",
  "gene_name": "Tripartite motif-containing protein 43B"
}